platelet degranulation [GO:0002576] (biological process) Sources: GOC:add Definition: The regulated exocytosis of secretory granules containing preformed mediators such as histamine and serotonin by a platelet. Relationships: is a type of regulated exocytosis [GO:0045055]; is a type of establishment of localization in cell [GO:0051649] Also known as: platelet exocytosis